{
  "gene_name": "Probable crossover junction endonuclease EME2",
  "term_id": "GO:0048476",
  "term_label": "Holliday junction resolvase complex",
  "gene_symbol": "EME2",
  "gene": "UniProtKB:A4GXA9"
}